{
  "term_label": "plasma membrane",
  "term_id": "GO:0005886",
  "gene": "UniProtKB:P78380",
  "gene_symbol": "OLR1",
  "gene_name": "Oxidized low-density lipoprotein receptor 1"
}